{
  "term_id": "GO:0030971",
  "term_label": "receptor tyrosine kinase binding",
  "gene_name": "Putative macrophage stimulating 1-like protein",
  "gene": "UniProtKB:Q2TV78",
  "gene_symbol": "MST1L"
}